{
  "term_id": "GO:0007409",
  "gene_symbol": "CELSR2",
  "gene": "UniProtKB:Q9HCU4",
  "term_label": "axonogenesis",
  "gene_name": "Cadherin EGF LAG seven-pass G-type receptor 2"
}